{
  "gene_symbol": "GRIK3",
  "gene_name": "Glutamate receptor ionotropic, kainate 3",
  "gene": "UniProtKB:Q13003",
  "term_label": "plasma membrane",
  "term_id": "GO:0005886"
}